{
  "gene_symbol": "SLC9B2",
  "gene_name": "Sodium_hydrogen exchanger 9B2",
  "gene": "UniProtKB:Q86UD5",
  "term_label": "Unknown cellular component",
  "term_id": "UNKNOWN:0003"
}